regulation of indoleacetic acid biosynthetic process via tryptophan [GO:1901996] (biological process) Definition: Any process that modulates the frequency, rate or extent of indoleacetic acid biosynthetic process via tryptophan. References: PMID:23377040 Sources: GOC:TermGenie Also known as: regulation of IAA biosynthetic process via tryptophan, regulation of indoleacetic acid anabolism via tryptophan, regulation of indoleacetic acid formation via tryptophan, regulation of indoleacetic acid synthesis via tryptophan Relationships: is a type of regulation of auxin biosynthetic process [GO:0010600]; is a type of GO:0090357; regulates indoleacetic acid biosynthetic process via tryptophan [GO:0009848] Subtypes: negative regulation of indoleacetic acid biosynthetic process via tryptophan [GO:1901997]